cyanelle outer membrane [GO:0036013] (cellular component) Sources: GOC:aa Definition: The outer, i.e. cytoplasm-facing, lipid bilayer of the cyanelle envelope. Relationships: is_a plastid outer membrane [GO:0009527]; is a type of cyanelle membrane [GO:0033113]